{
  "gene_symbol": "INVS",
  "term_label": "kidney development",
  "term_id": "GO:0001822",
  "gene": "UniProtKB:Q9Y283",
  "gene_name": "Inversin"
}